{
  "gene_name": "V-set and immunoglobulin domain-containing protein 4",
  "gene_symbol": "VSIG4",
  "term_label": "Unknown cellular component",
  "gene": "UniProtKB:Q9Y279",
  "term_id": "UNKNOWN:0003"
}